{
  "term_label": "gamma-butyrobetaine dioxygenase activity",
  "gene_symbol": "BBOX1",
  "gene_name": "Gamma-butyrobetaine dioxygenase",
  "gene": "UniProtKB:O75936",
  "term_id": "GO:0008336"
}